{
  "term_label": "rescue of stalled ribosome",
  "gene": "UniProtKB:O94822",
  "term_id": "GO:0072344",
  "gene_name": "E3 ubiquitin-protein ligase listerin",
  "gene_symbol": "LTN1"
}